organellar chromatophore thylakoid membrane [GO:0070118] (cellular component) Relationships: is a type of GO:0042651; is a type of GO:0070112; is part of organellar chromatophore thylakoid [GO:0070116] Also known as: Paulinella-type chromatophore thylakoid membrane Sources: GOC:mah Definition: The lipid bilayer membrane of any thylakoid within an organellar chromatophore.